olfactory bulb interneuron differentiation [GO:0021889] (biological process) Definition: The process in which a neuroblast acquires specialized features of an interneuron residing in the olfactory bulb. References: PMID:12626695 Sources: GOC:cls, GOC:dgh, GOC:dph, GOC:jid, GO_REF:0000021 Relationships: is a type of forebrain neuron differentiation [GO:0021879]; is part of olfactory bulb development [GO:0021772]